male pigmentation [GO:0048094] (biological process) Sources: GOC:jid Relationships: is a type of sex-specific pigmentation [GO:0048071]; is part of male sex differentiation [GO:0046661] Definition: Establishment of a pattern of pigment in males. Regulation: regulated by regulation of male pigmentation [GO:0048088]; negatively regulated by negative regulation of male pigmentation [GO:0048092]; positively regulated by positive regulation of male pigmentation [GO:0048093]